{
  "gene_symbol": "FGFBP3",
  "gene_name": "Fibroblast growth factor-binding protein 3",
  "gene": "UniProtKB:Q8TAT2",
  "term_id": "GO:0019838",
  "term_label": "growth factor binding"
}